adenosine salvage [GO:0006169] (biological process) Definition: Any process that generates adenosine, adenine riboside, from derivatives of it without de novo synthesis. Also known as: adenine, hypoxanthine and their nucleoside salvage Relationships: is a type of GO:0006166; is a type of adenosine biosynthetic process [GO:0046086] Sources: GOC:jl